{
  "gene_symbol": "OR8H2",
  "gene": "UniProtKB:Q8N162",
  "term_id": "UNKNOWN:0003",
  "gene_name": "Olfactory receptor 8H2",
  "term_label": "Unknown cellular component"
}